molybdenum cofactor sulfurtransferase activity [GO:0008265] (molecular function) References: PMID:11549764 Sources: RHEA:42636 Also known as: Mo-molybdopterin cofactor sulfurase activity, Mo-molybdopterin cofactor sulphurase activity, molybdopterin cofactor sulfurase activity, molybdopterin synthase sulfurylase activity Relationships: is a type of sulfurtransferase activity [GO:0016783] Definition: Catalysis of the reaction: AH2 + L-cysteine + Mo-molybdopterin = A + H2O + L-alanine + thio-Mo-molybdopterin.